{
  "term_id": "GO:0007416",
  "gene": "UniProtKB:Q8IZU9",
  "gene_symbol": "KIRREL3",
  "term_label": "synapse assembly",
  "gene_name": "Kin of IRRE-like protein 3"
}